{
  "gene": "UniProtKB:Q13885",
  "gene_symbol": "TUBB2A",
  "term_label": "neuron migration",
  "gene_name": "Tubulin beta-2A chain",
  "term_id": "GO:0001764"
}